{
  "gene": "UniProtKB:O95750",
  "term_label": "positive regulation of MAPK cascade",
  "term_id": "GO:0043410",
  "gene_name": "Fibroblast growth factor 19",
  "gene_symbol": "FGF19"
}